{
  "term_label": "protein serine/threonine kinase activity",
  "gene_name": "Serine_threonine-protein kinase ATR",
  "gene_symbol": "ATR",
  "term_id": "GO:0004674",
  "gene": "UniProtKB:Q13535"
}